{
  "term_id": "GO:0098921",
  "gene_symbol": "DAGLA",
  "gene": "UniProtKB:Q9Y4D2",
  "term_label": "retrograde trans-synaptic signaling by endocannabinoid",
  "gene_name": "Diacylglycerol lipase-alpha"
}